apoptotic process involved in metanephric nephron tubule development [GO:1900205] (biological process) Regulation: regulated by regulation of apoptotic process involved in metanephric nephron tubule development [GO:1900217]; negatively regulated by negative regulation of apoptotic process involved in metanephric nephron tubule development [GO:1900218]; positively regulated by positive regulation of apoptotic process involved in metanephric nephron tubule development [GO:1900219] References: PMID:17314325 Sources: GOC:TermGenie, GOC:mtg_kidney_jan10, GOC:yaf Relationships: is a type of apoptotic process involved in development [GO:1902742]; is part of metanephric nephron tubule development [GO:0072234] Definition: Any apoptotic process that is involved in metanephric nephron tubule development. Also known as: apoptotic cell death of metanephric nephron tubule development, apoptotic process of metanephric nephron tubule development, apoptotic programmed cell death of metanephric nephron tubule development, programmed cell death by apoptosis of metanephric nephron tubule development, apoptosis of metanephric nephron tubule development, apoptotic program of metanephric nephron tubule development, type I programmed cell death of metanephric nephron tubule development, signaling (initiator) caspase activity of metanephric nephron tubule development